{
  "gene_symbol": "SYNGR2",
  "gene_name": "Synaptogyrin-2",
  "gene": "UniProtKB:O43760",
  "term_id": "GO:0030672",
  "term_label": "synaptic vesicle membrane"
}